{
  "gene_symbol": "CA4",
  "term_id": "UNKNOWN:0002",
  "term_label": "Unknown biological process",
  "gene_name": "Carbonic anhydrase 4",
  "gene": "UniProtKB:P22748"
}